{
  "gene_name": "KIR2DL1 protein",
  "gene": "UniProtKB:A0A5K1VDZ0",
  "gene_symbol": "KIR2DL1",
  "term_id": "GO:0002767",
  "term_label": "immune response-inhibiting cell surface receptor signaling pathway"
}